{
  "gene_symbol": "GSTA5",
  "gene": "UniProtKB:Q7RTV2",
  "gene_name": "Glutathione S-transferase A5",
  "term_id": "GO:0004364",
  "term_label": "glutathione transferase activity"
}